{
  "gene_symbol": "TAFA5",
  "term_id": "GO:0001664",
  "gene_name": "Chemokine-like protein TAFA-5",
  "term_label": "G protein-coupled receptor binding",
  "gene": "UniProtKB:Q7Z5A7"
}